{
  "term_id": "UNKNOWN:0001",
  "gene": "UniProtKB:Q5HYI7",
  "gene_name": "Metaxin-3",
  "gene_symbol": "MTX3",
  "term_label": "Unknown molecular function"
}